{
  "gene": "UniProtKB:Q7Z4H7",
  "gene_symbol": "HAUS6",
  "term_label": "microtubule cytoskeleton organization",
  "gene_name": "HAUS augmin-like complex subunit 6",
  "term_id": "GO:0000226"
}